{
  "gene_symbol": "HLA-B",
  "term_label": "peptide antigen binding",
  "gene": "UniProtKB:P01889",
  "term_id": "GO:0042605",
  "gene_name": "HLA class I histocompatibility antigen, B alpha chain"
}